regulation of peptidyl-threonine phosphorylation [GO:0010799] (BP) Definition: Any process that modulates the frequency, rate or extent of peptidyl-threonine phosphorylation. Peptidyl-threonine phosphorylation is the phosphorylation of peptidyl-threonine to form peptidyl-O-phospho-L-threonine. Subtypes: positive regulation of peptidyl-threonine phosphorylation [GO:0010800], GO:0010801 Relationships: is a type of regulation of protein phosphorylation [GO:0001932]; regulates GO:0018107 Sources: GOC:dph, GOC:tb